{
  "gene": "UniProtKB:Q56P42",
  "term_label": "Unknown biological process",
  "gene_symbol": "PYDC2",
  "term_id": "UNKNOWN:0002",
  "gene_name": "Pyrin domain-containing protein 2"
}